negative regulation of cartilage development [GO:0061037] (biological process) Definition: Any process that decreases the rate, frequency, or extent of cartilage development, the process whose specific outcome is the progression of the cartilage over time, from its formation to the mature structure. Cartilage is a connective tissue dominated by extracellular matrix containing collagen type II and large amounts of proteoglycan, particularly chondroitin sulfate. Relationships: is a type of negative regulation of developmental process [GO:0051093]; is a type of GO:0051241; is a type of regulation of cartilage development [GO:0061035]; negatively regulates cartilage development [GO:0051216] Subtypes: negative regulation of chondrocyte differentiation [GO:0032331] Sources: GOC:dph